{
  "gene_symbol": "HOXC8",
  "term_id": "GO:0005634",
  "term_label": "nucleus",
  "gene_name": "Homeobox protein Hox-C8",
  "gene": "UniProtKB:P31273"
}